entry receptor-mediated virion attachment to host cell [GO:0098670] (biological process) References: PMID:18351291 Sources: VZ:3942 Relationships: is a type of GO:0046813 Definition: The process by which a virion attaches to a host cell by binding to a receptor on the host cell surface that mediates/triggers viral entry by endocytosis/pinocytosis or by inducing fusion/penetration. Also known as: viral attachment to host entry receptor Subtypes: receptor-mediated bacteriophage irreversible attachment to host cell [GO:0098002]